{
  "gene_name": "NACHT, LRR and PYD domains-containing protein 6",
  "gene": "UniProtKB:P59044",
  "term_id": "GO:0005737",
  "gene_symbol": "NLRP6",
  "term_label": "cytoplasm"
}